ventricular septum intermedium development [GO:0003282] (biological process) Sources: GOC:mtg_heart Relationships: is a type of ventricular septum development [GO:0003281] Definition: The progression of the ventricular septum intermedium over time, from its formation to the mature structure.